5-diphosphoinositol pentakisphosphate 6-kinase activity [GO:0000834] (molecular function) Relationships: is a type of GO:0000829 Also known as: inositol heptakisphosphate 6-kinase activity References: PMID:16429326 Sources: GOC:elh Definition: Catalysis of the reaction: ATP + 5-diphospho-1D-myo-inositol (1,2,3,4,6)pentakisphosphate = ADP + 5,6-bisdiphosphoinositol-1D-myo-inositol (1,2,3,4)tetrakisphosphate.